2-aminohexano-6-lactam racemase activity [GO:0047463] (molecular function) Definition: Catalysis of the reaction: L-2-aminohexano-6-lactam = D-2-aminohexano-6-lactam. Sources: EC:5.1.1.15, RHEA:14813 Relationships: is_a racemase and epimerase activity, acting on amino acids and derivatives [GO:0016855] Also known as: 2-amino-hexano-6-lactam racemase activity, alpha-amino-epsilon-caprolactam racemase activity